{
  "term_label": "DNA-binding transcription factor activity, RNA polymerase II-specific",
  "term_id": "GO:0000981",
  "gene": "UniProtKB:Q9BWM5",
  "gene_name": "Zinc finger protein 416",
  "gene_symbol": "ZNF416"
}